regulation of systemic arterial blood pressure by acetylcholine [GO:0003068] (biological process) Relationships: is a type of GO:0003070 Also known as: blood pressure regulation by acetylcholine Sources: GOC:mtg_cardio, GOC:rl Definition: The regulation of blood pressure mediated by acetylcholine signaling. Acetylcholine is an acetic acid ester of the organic base choline and functions as a neurotransmitter.